{
  "term_id": "GO:0007411",
  "term_label": "axon guidance",
  "gene_symbol": "SEMA3E",
  "gene": "UniProtKB:O15041",
  "gene_name": "Semaphorin-3E"
}